response to mannitol [GO:0010555] (biological process) Also known as: response to mannitol stimulus Definition: Any process that results in a change in state or activity of a cell or an organism (in terms of movement, secretion, enzyme production, gene expression, etc.) as a result of a mannitol stimulus. Subtypes: cellular response to mannitol stimulus [GO:0071325] References: PMID:17999646 Relationships: is a type of response to carbohydrate [GO:0009743]